{
  "gene": "UniProtKB:Q9NT99",
  "gene_name": "Leucine-rich repeat-containing protein 4B",
  "term_label": "postsynaptic density membrane",
  "gene_symbol": "LRRC4B",
  "term_id": "GO:0098839"
}